{
  "gene_symbol": "GAS8",
  "term_id": "GO:0005794",
  "term_label": "Golgi apparatus",
  "gene_name": "Dynein regulatory complex subunit 4",
  "gene": "UniProtKB:O95995"
}